{
  "gene": "UniProtKB:Q16816",
  "gene_symbol": "PHKG1",
  "gene_name": "Phosphorylase b kinase gamma catalytic chain, skeletal muscle_heart isoform",
  "term_label": "phosphorylase kinase activity",
  "term_id": "GO:0004689"
}